ATPase-coupled ion transmembrane transporter activity [GO:0042625] (molecular function) Relationships: is a type of GO:0042626 Definition: Enables the transfer of an ion from one side of a membrane to the other, driven by the reaction: ATP + H2O = ADP + phosphate. Subtypes: ATPase activity, coupled to transmembrane movement of ions, rotational mechanism [GO:0044769], ATPase coupled ion transmembrane transporter activity involved in regulation of presynaptic membrane potential [GO:0099521], ATPase coupled ion transmembrane transporter activity involved in regulation of postsynaptic membrane potential [GO:0099581] Also known as: ATP-dependent ion transmembrane transporter activity, ATPase activity, coupled to transmembrane movement of ions, ATPase coupled ion transmembrane transporter activity Sources: GOC:jl, GOC:mtg_transport, ISBN:0815340729